regulation of convergent extension involved in rhombomere morphogenesis [GO:1904133] (biological process) Subtypes: negative regulation of convergent extension involved in rhombomere morphogenesis [GO:1904134], GO:1904135 References: PMID:24892953 Sources: GOC:TermGenie, GOC:dph, GO_REF:0000058 Relationships: is a type of regulation of convergent extension involved in gastrulation [GO:1904103]; regulates convergent extension involved in rhombomere morphogenesis [GO:1904125] Definition: Any process that modulates the frequency, rate or extent of convergent extension involved in rhombomere morphogenesis.